striated muscle cell differentiation [GO:0051146] (biological process) Subtypes: myotube differentiation [GO:0014902], cardiac muscle cell differentiation [GO:0055007] Relationships: is a type of muscle cell differentiation [GO:0042692] Sources: CL:0000737, GOC:ai Regulation: regulated by regulation of striated muscle cell differentiation [GO:0051153]; negatively regulated by negative regulation of striated muscle cell differentiation [GO:0051154]; RO_0002213 by positive regulation of striated muscle cell differentiation [GO:0051155] Also known as: voluntary muscle cell differentiation Definition: The process in which a relatively unspecialized cell acquires specialized features of a striated muscle cell; striated muscle fibers are divided by transverse bands into striations, and cardiac and voluntary muscle are types of striated muscle.